{
  "gene": "UniProtKB:P31751",
  "term_label": "insulin receptor signaling pathway",
  "term_id": "GO:0008286",
  "gene_name": "RAC-beta serine_threonine-protein kinase",
  "gene_symbol": "AKT2"
}